cinnamoyl-CoA reductase activity [GO:0016621] (molecular function) Also known as: cinnamoyl CoA reductase activity, cinnamaldehyde:NADP+ oxidoreductase (CoA-cinnamoylating), cinnamoyl-CoA:NADPH reductase activity, cinnamoyl-coenzyme A reductase activity, feruloyl coenzyme A reductase activity, feruloyl-CoA reductase activity, ferulyl-CoA reductase activity, p-hydroxycinnamoyl coenzyme A reductase activity Sources: EC:1.2.1.44 Definition: Catalysis of the reaction: cinnamaldehyde + CoA + NADP+ = cinnamoyl-CoA + NADPH + H+. Relationships: is a type of oxidoreductase activity, acting on the aldehyde or oxo group of donors, NAD or NADP as acceptor [GO:0016620]